{
  "gene_name": "T cell receptor beta variable 6-5",
  "gene_symbol": "TRBV6-5",
  "term_id": "GO:0005886",
  "term_label": "plasma membrane",
  "gene": "UniProtKB:A0A0K0K1A5"
}